{
  "term_label": "Unknown molecular function",
  "gene_symbol": "SAPCD2",
  "gene": "UniProtKB:Q86UD0",
  "gene_name": "Suppressor APC domain-containing protein 2",
  "term_id": "UNKNOWN:0001"
}